{
  "term_id": "GO:0005940",
  "gene_symbol": "SEPTIN5",
  "gene_name": "Septin-5",
  "gene": "UniProtKB:Q99719",
  "term_label": "septin ring"
}